{
  "term_id": "UNKNOWN:0003",
  "gene_symbol": "FBXO36",
  "term_label": "Unknown cellular component",
  "gene_name": "F-box only protein 36",
  "gene": "UniProtKB:Q8NEA4"
}